cyclin A1-CDK2 complex [GO:0097123] (cellular component) Relationships: is a type of cyclin-dependent protein kinase holoenzyme complex [GO:0000307] Definition: A protein complex consisting of cyclin A1 and cyclin-dependent kinase 2 (CDK2). Cyclins are characterized by periodicity in protein abundance throughout the cell cycle. Cyclin-dependent kinases represent a family of serine/threonine protein kinases that become active upon binding to a cyclin regulatory partner. References: PMID:15935619 Sources: GOC:so